{
  "gene": "UniProtKB:A7MBM2",
  "gene_symbol": "DISP2",
  "gene_name": "Protein dispatched homolog 2",
  "term_label": "membrane",
  "term_id": "GO:0016020"
}